{
  "term_id": "GO:0006816",
  "gene_name": "Transient receptor potential cation channel subfamily M member 7",
  "gene_symbol": "TRPM7",
  "gene": "UniProtKB:Q96QT4",
  "term_label": "calcium ion transport"
}